inulin catabolic process [GO:1902927] (biological process) Relationships: is a type of GO:0010147 Definition: The chemical reactions and pathways resulting in the breakdown of inulin. References: PMID:23104410 Sources: GOC:TermGenie, GO_REF:0000068 Note: SUC2 in S. cerevisiae strain JZ1C in PMID:23104410. Also known as: inulin breakdown, inulin catabolism, inulin degradation